{
  "gene_name": "ATP-dependent DNA helicase Q5",
  "term_label": "four-way junction helicase activity",
  "gene": "UniProtKB:O94762",
  "term_id": "GO:0009378",
  "gene_symbol": "RECQL5"
}